{
  "gene": "UniProtKB:Q86TB9",
  "gene_symbol": "PATL1",
  "gene_name": "Protein PAT1 homolog 1",
  "term_label": "P-body assembly",
  "term_id": "GO:0033962"
}